{
  "gene": "UniProtKB:P40426",
  "term_id": "GO:0001654",
  "gene_symbol": "PBX3",
  "term_label": "eye development",
  "gene_name": "Pre-B-cell leukemia transcription factor 3"
}